{
  "gene_name": "NACHT, LRR and PYD domains-containing protein 5",
  "term_id": "GO:0005739",
  "gene": "UniProtKB:P59047",
  "gene_symbol": "NLRP5",
  "term_label": "mitochondrion"
}